{
  "gene": "UniProtKB:Q9P2D1",
  "gene_symbol": "CHD7",
  "term_id": "GO:0021545",
  "gene_name": "Chromodomain-helicase-DNA-binding protein 7",
  "term_label": "cranial nerve development"
}